{
  "term_label": "plasma membrane",
  "gene_name": "Rap guanine nucleotide exchange factor 1",
  "term_id": "GO:0005886",
  "gene": "UniProtKB:Q13905",
  "gene_symbol": "RAPGEF1"
}